{
  "term_label": "endosome to lysosome transport",
  "gene": "UniProtKB:Q8N612",
  "gene_name": "FHF complex subunit HOOK-interacting protein 1B",
  "gene_symbol": "FHIP1B",
  "term_id": "GO:0008333"
}